{
  "term_id": "GO:0005886",
  "gene_symbol": "PROKR2",
  "gene_name": "Prokineticin receptor 2",
  "term_label": "plasma membrane",
  "gene": "UniProtKB:Q8NFJ6"
}